{
  "term_label": "DNA topological change",
  "gene_name": "DNA topoisomerase 3-beta-1",
  "term_id": "GO:0006265",
  "gene": "UniProtKB:O95985",
  "gene_symbol": "TOP3B"
}